{
  "gene_name": "PDZ and LIM domain protein 1",
  "term_id": "GO:0007507",
  "gene": "UniProtKB:O00151",
  "term_label": "heart development",
  "gene_symbol": "PDLIM1"
}